{
  "gene": "UniProtKB:Q6ZS30",
  "term_id": "UNKNOWN:0002",
  "gene_name": "Neurobeachin-like protein 1",
  "term_label": "Unknown biological process",
  "gene_symbol": "NBEAL1"
}